{
  "gene_symbol": "PTGES3",
  "gene": "UniProtKB:Q15185",
  "gene_name": "Prostaglandin E synthase 3",
  "term_label": "prostaglandin-E synthase activity",
  "term_id": "GO:0050220"
}